double-strand break repair via classical nonhomologous end joining [GO:0097680] (biological process) Relationships: is a type of double-strand break repair via nonhomologous end joining [GO:0006303] Definition: An instance of double-strand break repair via nonhomologous end joining that requires a number of factors important for V(D)J recombination, including the KU70/80 heterodimer (KU), XRCC4, ligase IV, and DNA-PKcs in mammals. It does not produce translocations (as opposed to the alternative nonhomologous end joining). References: PMID:18584027 Sources: GOC:rph Also known as: canonical nonhomologous end joining, C-NHEJ